{
  "term_label": "Unknown cellular component",
  "gene_name": "Rho guanine nucleotide exchange factor 15",
  "term_id": "UNKNOWN:0003",
  "gene_symbol": "ARHGEF15",
  "gene": "UniProtKB:O94989"
}